{
  "gene_name": "Kelch-like protein 20",
  "term_id": "GO:0005737",
  "gene_symbol": "KLHL20",
  "gene": "UniProtKB:Q9Y2M5",
  "term_label": "cytoplasm"
}